{
  "term_id": "UNKNOWN:0003",
  "gene_symbol": "DUSP28",
  "gene": "UniProtKB:Q4G0W2",
  "gene_name": "Dual specificity phosphatase 28",
  "term_label": "Unknown cellular component"
}